{
  "term_id": "UNKNOWN:0001",
  "term_label": "Unknown molecular function",
  "gene": "UniProtKB:Q9P1J3",
  "gene_symbol": "DHRS4-AS1",
  "gene_name": "Putative uncharacterized protein DHRS4-AS1"
}